{
  "gene": "UniProtKB:Q6NYC8",
  "gene_name": "Phostensin",
  "term_label": "Unknown biological process",
  "gene_symbol": "PPP1R18",
  "term_id": "UNKNOWN:0002"
}